{
  "gene_name": "Kelch-like protein 30",
  "term_label": "Cul3-RING ubiquitin ligase complex",
  "term_id": "GO:0031463",
  "gene": "UniProtKB:Q0D2K2",
  "gene_symbol": "KLHL30"
}